regulation of carbohydrate biosynthetic process [GO:0043255] (biological process) Also known as: regulation of carbohydrate anabolism, regulation of carbohydrate biosynthesis, regulation of carbohydrate formation, regulation of carbohydrate synthesis Definition: Any process that modulates the frequency, rate or extent of the chemical reactions and pathways resulting in the formation of carbohydrates. Sources: GOC:jl Relationships: is a type of regulation of carbohydrate metabolic process [GO:0006109]; is a type of regulation of biosynthetic process [GO:0009889]; regulates carbohydrate biosynthetic process [GO:0016051] Subtypes: GO:0006111, regulation of photosynthesis, dark reaction [GO:0010110], regulation of glucosinolate biosynthetic process [GO:0010439], regulation of inositol phosphate biosynthetic process [GO:0010919], regulation of polysaccharide biosynthetic process [GO:0032885], regulation of raffinose biosynthetic process [GO:1900091], GO:1903534, regulation of L-ascorbic acid biosynthetic process [GO:2000082]